{
  "gene": "UniProtKB:Q15771",
  "term_label": "GTPase activity",
  "gene_symbol": "RAB30",
  "gene_name": "Ras-related protein Rab-30",
  "term_id": "GO:0003924"
}